cellular response to oxygen-glucose deprivation [GO:0090650] (biological process) Definition: Any process that results in a change in state or activity of a cell (in terms of movement, secretion, enzyme production, gene expression, etc.) as a result of the deprivation of oxygen and glucose. References: PMID:21525936 Sources: GOC:sl Also known as: cellular response to OGD Relationships: is a type of cellular response to nutrient levels [GO:0031669]; is a type of cellular response to decreased oxygen levels [GO:0036294]; is a type of response to oxygen-glucose deprivation [GO:0090649]